negative regulation of tolerance induction to self antigen [GO:0002650] (biological process) Relationships: is a type of negative regulation of tolerance induction [GO:0002644]; is a type of regulation of tolerance induction to self antigen [GO:0002649]; negatively regulates tolerance induction to self antigen [GO:0002513] Also known as: down regulation of tolerance induction to self antigen, down-regulation of tolerance induction to self antigen, downregulation of tolerance induction to self antigen, inhibition of tolerance induction to self antigen Sources: GOC:add Definition: Any process that stops, prevents, or reduces the frequency, rate, or extent of tolerance induction to self antigen.